substance P receptor binding [GO:0031835] (molecular function) Sources: GOC:mah, GOC:nln Definition: Binding to a substance P receptor. Relationships: is a type of neurokinin receptor binding [GO:0031834] Also known as: neurokinin-1 receptor binding, substance P receptor ligand